{
  "gene_symbol": "ALPP",
  "term_label": "Unknown biological process",
  "term_id": "UNKNOWN:0002",
  "gene": "UniProtKB:P05187",
  "gene_name": "Alkaline phosphatase, placental type"
}